{
  "term_label": "transcription corepressor activity",
  "gene_symbol": "ID2",
  "term_id": "GO:0003714",
  "gene_name": "DNA-binding protein inhibitor ID-2",
  "gene": "UniProtKB:Q02363"
}